{
  "gene": "UniProtKB:Q04446",
  "gene_symbol": "GBE1",
  "term_label": "cytoplasm",
  "gene_name": "1,4-alpha-glucan-branching enzyme",
  "term_id": "GO:0005737"
}